{
  "gene": "UniProtKB:O60911",
  "term_label": "extracellular space",
  "term_id": "GO:0005615",
  "gene_symbol": "CTSV",
  "gene_name": "Cathepsin L2"
}